{
  "term_label": "structural constituent of chromatin",
  "gene_symbol": "H2BC18",
  "gene": "UniProtKB:Q5QNW6",
  "term_id": "GO:0030527",
  "gene_name": "Histone H2B type 2-F"
}